{
  "gene_symbol": "TUBA1C",
  "term_label": "microtubule",
  "gene": "UniProtKB:Q9BQE3",
  "term_id": "GO:0005874",
  "gene_name": "Tubulin alpha-1C chain"
}